{
  "term_label": "G protein-coupled receptor activity",
  "gene_name": "Probable G-protein coupled receptor 19",
  "term_id": "GO:0004930",
  "gene_symbol": "GPR19",
  "gene": "UniProtKB:Q15760"
}